negative regulation of protein kinase activity by regulation of protein phosphorylation [GO:0044387] (biological process) Relationships: is a type of negative regulation of protein kinase activity [GO:0006469] Sources: GOC:jl Definition: The stopping, prevention, or reduction in frequency, rate or extent of protein kinase activity as a result of regulating the phosphorylation status of that protein kinase.